{
  "term_id": "GO:0005524",
  "gene_symbol": "PGK2",
  "term_label": "ATP binding",
  "gene": "UniProtKB:P07205",
  "gene_name": "Phosphoglycerate kinase 2"
}